{
  "gene_name": "Arachidonate 5-lipoxygenase-activating protein",
  "term_id": "GO:0019370",
  "gene_symbol": "ALOX5AP",
  "gene": "UniProtKB:P20292",
  "term_label": "leukotriene biosynthetic process"
}